nicotine dehydrogenase activity [GO:0018535] (molecular function) Definition: Catalysis of the reaction: nicotine + acceptor + H2O = (S)-6-hydroxynicotine + reduced acceptor. Sources: EC:1.5.99.4 Relationships: is a type of oxidoreductase activity, acting on the CH-NH group of donors [GO:0016645] Also known as: D-nicotine oxidase activity, nicotine oxidase activity, nicotine:(acceptor) 6-oxidoreductase (hydroxylating), nicotine:acceptor 6-oxidoreductase (hydroxylating)